negative regulation of protein modification by small protein conjugation or removal [GO:1903321] (biological process) Definition: Any process that stops, prevents or reduces the frequency, rate or extent of protein modification by small protein conjugation or removal. Sources: GOC:TermGenie, GOC:vw, GO_REF:0000058 Also known as: down regulation of protein modification by small protein conjugation or removal, down-regulation of protein modification by small protein conjugation or removal, downregulation of protein modification by small protein conjugation or removal, inhibition of protein modification by small protein conjugation or removal Relationships: is a type of GO:1901874; is a type of regulation of protein modification by small protein conjugation or removal [GO:1903320]; negatively regulates protein modification by small protein conjugation or removal [GO:0070647] Subtypes: negative regulation of protein ubiquitination [GO:0031397], negative regulation of protein sumoylation [GO:0033234], negative regulation of protein desumoylation [GO:0060190], negative regulation of protein deubiquitination [GO:0090086], negative regulation of protein neddylation [GO:2000435]